{
  "term_label": "proteasome-mediated ubiquitin-dependent protein catabolic process",
  "gene_name": "Kelch-like protein 1",
  "term_id": "GO:0043161",
  "gene_symbol": "KLHL1",
  "gene": "UniProtKB:Q9NR64"
}